apoptotic signaling pathway [GO:0097190] (biological process) Regulation: regulated by regulation of apoptotic signaling pathway [GO:2001233]; negatively regulated by negative regulation of apoptotic signaling pathway [GO:2001234]; positively regulated by positive regulation of apoptotic signaling pathway [GO:2001235] Subtypes: GO:0008626, hormone-mediated apoptotic signaling pathway [GO:0008628], extrinsic apoptotic signaling pathway [GO:0097191], intrinsic apoptotic signaling pathway [GO:0097193] Sources: GOC:mtg_apoptosis Note: This term can be used to annotate gene products involved in apoptotic events happening downstream of the cross-talk point between the extrinsic and intrinsic apoptotic pathways. The cross-talk starts when caspase-8 cleaves Bid and truncated Bid interacts with mitochondria. From this point on it is not possible to distinguish between extrinsic and intrinsic pathways. Definition: The series of molecular signals which triggers the apoptotic death of a cell. The pathway starts with reception of a signal, and ends when the execution phase of apoptosis is triggered. Relationships: is a type of signal transduction [GO:0007165]; is part of apoptotic process [GO:0006915] Also known as: apoptotic signalling pathway, induction of apoptosis by extracellular signals